{
  "term_id": "GO:0019901",
  "term_label": "protein kinase binding",
  "gene_name": "Putative speedy protein E13",
  "gene": "UniProtKB:A0A494C0Z2",
  "gene_symbol": "SPDYE13"
}